emericellamide A catabolic process [GO:1900616] (biological process) Definition: The chemical reactions and pathways resulting in the breakdown of emericellamide A. Sources: GOC:TermGenie, GOC:di Also known as: emericellamide A breakdown, emericellamide A catabolism, emericellamide A degradation Relationships: is a type of GO:1900556